{
  "term_label": "stimulatory C-type lectin receptor signaling pathway",
  "gene_symbol": "KLRC3",
  "gene": "UniProtKB:Q07444",
  "gene_name": "NKG2-E type II integral membrane protein",
  "term_id": "GO:0002223"
}